{
  "gene_symbol": "BMPR2",
  "gene_name": "Bone morphogenetic protein receptor type-2",
  "term_id": "GO:0005886",
  "term_label": "plasma membrane",
  "gene": "UniProtKB:Q13873"
}